very long-chain fatty acid biosynthetic process [GO:0042761] (biological process) Also known as: very-long-chain fatty acid anabolism, very-long-chain fatty acid biosynthesis, very-long-chain fatty acid biosynthetic process, very-long-chain fatty acid formation, very-long-chain fatty acid synthesis Relationships: is a type of very long-chain fatty acid metabolic process [GO:0000038]; is_a GO:0006633 References: PMID:7744868 Definition: The chemical reactions and pathways resulting in the formation of a very long-chain fatty acid. A very long-chain fatty acid has an aliphatic tail containing more than 22 carbons. Note: While there is not universal consensus on the lengths of short-, medium-, long- and very-long-chain fatty acids, the GO uses the definitions in ChEBI (see CHEBI:26666, CHEBI:59554, CHEBI:15904 and CHEBI:27283).